{
  "gene_name": "Acrosin",
  "gene_symbol": "ACR",
  "term_id": "UNKNOWN:0003",
  "term_label": "Unknown cellular component",
  "gene": "UniProtKB:P10323"
}